{
  "term_label": "odorant binding",
  "term_id": "GO:0005549",
  "gene_name": "Olfactory receptor 10J3",
  "gene_symbol": "OR10J3",
  "gene": "UniProtKB:Q5JRS4"
}